{
  "gene_symbol": "FOLR1",
  "gene_name": "Folate receptor alpha",
  "term_label": "signaling receptor activity",
  "gene": "UniProtKB:P15328",
  "term_id": "GO:0038023"
}